{
  "term_id": "GO:0003865",
  "gene": "UniProtKB:P31213",
  "gene_name": "3-oxo-5-alpha-steroid 4-dehydrogenase 2",
  "gene_symbol": "SRD5A2",
  "term_label": "3-oxo-5-alpha-steroid 4-dehydrogenase activity"
}